rolling circle double-stranded viral DNA replication [GO:0039683] (biological process) Relationships: is a type of GO:0039682 Sources: GOC:bf, GOC:jl, VZ:2676 Definition: A rolling circle viral DNA replication that begins with a double-stranded viral DNA genome. Also known as: dsDNA rolling circle replication